{
  "gene_name": "Lupus La protein",
  "term_id": "GO:0045727",
  "term_label": "positive regulation of translation",
  "gene_symbol": "SSB",
  "gene": "UniProtKB:P05455"
}